tubulin-dependent ATPase activity [GO:0070463] (molecular function) Definition: Catalysis of the reaction: ATP + H2O = ADP + phosphate. This reaction requires the presence of a tubulin dimer to accelerate release of ADP and phosphate. References: PMID:16906148 Sources: GOC:mah Also known as: tubulin-activated ATPase activity Relationships: is_a ATP-dependent activity [GO:0140657]